folic acid-containing compound metabolic process [GO:0006760] (biological process) Sources: GOC:ai, GOC:mah Also known as: folate and derivative metabolic process, folate and derivative metabolism, folate-containing compound metabolic process, folate-containing compound metabolism, folic acid and derivative metabolic process, folic acid and derivative metabolism, folic acid-containing compound metabolism, vitamin B9 and derivative metabolic process, vitamin B9 and derivative metabolism, vitamin M and derivative metabolic process, vitamin M and derivative metabolism Relationships: is a type of GO:0006575; is a type of pteridine-containing compound metabolic process [GO:0042558] Definition: The chemical reactions and pathways involving a folic acid-containing compound, i.e. any of a group of heterocyclic compounds based on the pteroic acid skeleton conjugated with one or more L-glutamic acid or L-glutamate units. Subtypes: folic acid-containing compound biosynthetic process [GO:0009396], folic acid-containing compound catabolic process [GO:0009397], dihydrofolate metabolic process [GO:0046452], tetrahydrofolate metabolic process [GO:0046653], GO:0046655, tetrahydrofolylpolyglutamate metabolic process [GO:0046900]